{
  "term_label": "cytoplasm",
  "gene": "UniProtKB:Q9UBC2",
  "gene_name": "Epidermal growth factor receptor substrate 15-like 1",
  "gene_symbol": "EPS15L1",
  "term_id": "GO:0005737"
}